{
  "term_id": "GO:0050727",
  "term_label": "regulation of inflammatory response",
  "gene_symbol": "GGT2P",
  "gene": "UniProtKB:P36268",
  "gene_name": "Inactive glutathione hydrolase 2"
}